{
  "term_id": "UNKNOWN:0003",
  "gene_name": "Zinc finger protein 562",
  "gene": "UniProtKB:Q6V9R5",
  "gene_symbol": "ZNF562",
  "term_label": "Unknown cellular component"
}